{
  "gene": "UniProtKB:O95935",
  "gene_symbol": "TBX18",
  "gene_name": "T-box transcription factor TBX18",
  "term_id": "GO:0000785",
  "term_label": "chromatin"
}